{
  "term_id": "GO:0000981",
  "gene": "UniProtKB:Q9NQB0",
  "term_label": "DNA-binding transcription factor activity, RNA polymerase II-specific",
  "gene_name": "Transcription factor 7-like 2",
  "gene_symbol": "TCF7L2"
}